{
  "gene_name": "Small ubiquitin-related modifier 2",
  "gene_symbol": "SUMO2",
  "term_label": "nucleus",
  "term_id": "GO:0005634",
  "gene": "UniProtKB:P61956"
}